{
  "gene_symbol": "DLL3",
  "gene_name": "Delta-like protein 3",
  "term_id": "GO:0005112",
  "term_label": "Notch binding",
  "gene": "UniProtKB:Q9NYJ7"
}